{
  "gene_name": "Chorionic somatomammotropin hormone-like 1",
  "term_label": "growth hormone receptor binding",
  "term_id": "GO:0005131",
  "gene": "UniProtKB:Q14406",
  "gene_symbol": "CSHL1"
}